spermidine biosynthetic process [GO:0008295] (biological process) Also known as: spermidine anabolism, spermidine biosynthesis, spermidine formation, spermidine synthesis Definition: The chemical reactions and pathways resulting in the formation of spermidine, N-(3-aminopropyl)-1,4-diaminobutane. Relationships: is a type of polyamine biosynthetic process [GO:0006596]; is a type of GO:0008216 Sources: GOC:go_curators, ISBN:0198506732 Regulation: regulated by regulation of spermidine biosynthetic process [GO:1901304]; negatively regulated by negative regulation of spermidine biosynthetic process [GO:1901305]; positively regulated by positive regulation of spermidine biosynthetic process [GO:1901307]